endoplasmic reticulum membrane fusion [GO:0016320] (biological process) Definition: The joining of 2 or more lipid bilayer membranes that surround the endoplasmic reticulum. Also known as: ER membrane fusion Sources: GOC:elh, GOC:jid Relationships: is a type of endoplasmic reticulum organization [GO:0007029]; is a type of endoplasmic reticulum membrane organization [GO:0090158]; is a type of GO:0090174